{
  "gene_symbol": "ADAD2",
  "term_label": "RNA processing",
  "term_id": "GO:0006396",
  "gene": "UniProtKB:Q8NCV1",
  "gene_name": "Adenosine deaminase domain-containing protein 2"
}